{
  "gene_symbol": "EZR",
  "term_id": "GO:0008360",
  "term_label": "regulation of cell shape",
  "gene": "UniProtKB:P15311",
  "gene_name": "Ezrin"
}